{
  "gene_name": "T-box transcription factor TBX6",
  "term_id": "GO:0000978",
  "gene": "UniProtKB:O95947",
  "gene_symbol": "TBX6",
  "term_label": "RNA polymerase II cis-regulatory region sequence-specific DNA binding"
}